{
  "gene_name": "E3 ubiquitin-protein ligase TRIM7",
  "term_label": "cytoplasm",
  "gene_symbol": "TRIM7",
  "gene": "UniProtKB:Q9C029",
  "term_id": "GO:0005737"
}